{
  "term_id": "UNKNOWN:0001",
  "gene_name": "Lysosomal-associated transmembrane protein 4A",
  "gene_symbol": "LAPTM4A",
  "gene": "UniProtKB:Q15012",
  "term_label": "Unknown molecular function"
}